{
  "gene_name": "Sarcoma antigen 1",
  "gene": "UniProtKB:Q9NXZ1",
  "term_id": "GO:0032039",
  "gene_symbol": "SAGE1",
  "term_label": "integrator complex"
}